{
  "term_id": "GO:0005246",
  "term_label": "calcium channel regulator activity",
  "gene": "UniProtKB:Q8IYK8",
  "gene_symbol": "REM2",
  "gene_name": "GTP-binding protein REM 2"
}